{
  "term_label": "serine-type endopeptidase activity",
  "gene": "UniProtKB:P48740",
  "gene_symbol": "MASP1",
  "gene_name": "Mannan-binding lectin serine protease 1",
  "term_id": "GO:0004252"
}